noncyclic photosynthetic phosphorylation [GO:0009779] (biological process) Relationships: is a type of photosynthetic phosphorylation [GO:0009777] Sources: ISBN:0198547684 Definition: A photosynthetic phosphorylation process in which ATP synthesis is linked to the transport of electrons from water to NADP+ with the production of NADPH and dioxygen (O2). Involves photosystem I and photosystem II.